spine mat [GO:0097448] (cellular component) Definition: A configuration of neuron spines found on ciliary ganglion neurons in the embryonic and adult brain consisting of patches of closely spaced spines lying flat against the soma. References: PMID:10818137 Sources: NIF_Subcellular:sao2128156969 Relationships: is a type of cellular anatomical structure [GO:0110165]; has part neuron spine [GO:0044309]